gamma-curcumene synthase activity [GO:0102064] (molecular function) Relationships: is a type of carbon-oxygen lyase activity, acting on phosphates [GO:0016838] Definition: Catalysis of the reaction: 2-trans,6-trans-farnesyl diphosphate = gamma-curcumene + diphosphoric acid. Sources: EC:4.2.3.94, GOC:pz